{
  "term_label": "nucleoplasm",
  "gene": "UniProtKB:Q9H8W5",
  "term_id": "GO:0005654",
  "gene_name": "E3 ubiquitin-protein ligase TRIM45",
  "gene_symbol": "TRIM45"
}